{
  "term_id": "GO:0072659",
  "gene": "UniProtKB:Q3MJ13",
  "gene_name": "WD repeat-containing protein 72",
  "term_label": "protein localization to plasma membrane",
  "gene_symbol": "WDR72"
}